{
  "gene": "UniProtKB:Q14687",
  "gene_symbol": "GSE1",
  "term_id": "UNKNOWN:0001",
  "gene_name": "Genetic suppressor element 1",
  "term_label": "Unknown molecular function"
}